SRP-dependent cotranslational protein targeting to membrane, translocation [GO:0006616] (biological process) Relationships: is a type of GO:0065002; is part of SRP-dependent cotranslational protein targeting to membrane [GO:0006614] Sources: ISBN:0716731363 Definition: The process during cotranslational membrane targeting wherein proteins move across a membrane. SRP and its receptor initiate the transfer of the nascent chain across the endoplasmic reticulum (ER) membrane; they then dissociate from the chain, which is transferred to a set of transmembrane proteins, collectively called the translocon. Once the nascent chain translocon complex is assembled, the elongating chain passes directly from the large ribosomal subunit into the centers of the translocon, a protein-lined channel within the membrane. The growing chain is never exposed to the cytosol and does not fold until it reaches the ER lumen. Also known as: ER translocation, SRP-dependent cotranslational membrane targeting, translocation, SRP-dependent cotranslational protein-membrane targeting, translocation, translocation during SRP-dependent cotranslational protein targeting to membrane